{
  "gene": "UniProtKB:Q8TAT5",
  "gene_symbol": "NEIL3",
  "gene_name": "Endonuclease 8-like 3",
  "term_label": "base-excision repair",
  "term_id": "GO:0006284"
}